{
  "gene": "UniProtKB:Q9P2D1",
  "term_label": "chromatin",
  "term_id": "GO:0000785",
  "gene_symbol": "CHD7",
  "gene_name": "Chromodomain-helicase-DNA-binding protein 7"
}